{
  "term_label": "cytoplasm",
  "term_id": "GO:0005737",
  "gene": "UniProtKB:P11055",
  "gene_name": "Myosin-3",
  "gene_symbol": "MYH3"
}